{
  "gene": "UniProtKB:P43080",
  "gene_name": "Guanylyl cyclase-activating protein 1",
  "term_id": "GO:0005509",
  "gene_symbol": "GUCA1A",
  "term_label": "calcium ion binding"
}